{
  "term_id": "GO:0005634",
  "gene_name": "Krueppel-like factor 5",
  "term_label": "nucleus",
  "gene": "UniProtKB:Q13887",
  "gene_symbol": "KLF5"
}